{
  "gene_symbol": "FNDC10",
  "gene": "UniProtKB:F2Z333",
  "term_id": "UNKNOWN:0003",
  "term_label": "Unknown cellular component",
  "gene_name": "Fibronectin type III domain-containing protein 10"
}